{
  "term_label": "negative regulation of TORC1 signaling",
  "gene_symbol": "KPTN",
  "gene_name": "KICSTOR complex protein kaptin",
  "gene": "UniProtKB:Q9Y664",
  "term_id": "GO:1904262"
}